{
  "gene_name": "Putative protein N-methyltransferase FAM86B2",
  "term_label": "protein-containing complex",
  "gene_symbol": "FAM86B2",
  "gene": "UniProtKB:P0C5J1",
  "term_id": "GO:0032991"
}